inhibition of acetylcholine uptake [GO:0051634] (biological process) Definition: Any process that prevents the activation of the directed movement of acetylcholine into a cell. Sources: GOC:ai Also known as: inhibition of acetylcholine import Relationships: is a type of GO:0051609; is a type of negative regulation of acetylcholine uptake [GO:0051632]